{
  "gene": "UniProtKB:Q13541",
  "gene_symbol": "EIF4EBP1",
  "term_id": "GO:0005829",
  "term_label": "cytosol",
  "gene_name": "Eukaryotic translation initiation factor 4E-binding protein 1"
}